protein localization to chromosome, centromeric region [GO:0071459] (biological process) Also known as: protein localisation to chromosome, centromeric region, protein localization to centromere, protein localization to chromosome, centric region Subtypes: protein localization to kinetochore [GO:0034501], protein localization to CENP-A containing chromatin [GO:0061644], protein localization to pericentric heterochromatin [GO:1902682] Relationships: is a type of protein localization to chromosome [GO:0034502] Definition: Any process in which a protein is transported to, or maintained at, the centromeric region of a chromosome. Sources: GOC:mah